{
  "term_id": "GO:1902495",
  "gene_symbol": "HTR3E",
  "term_label": "transmembrane transporter complex",
  "gene_name": "5-hydroxytryptamine receptor 3E",
  "gene": "UniProtKB:A5X5Y0"
}